formyl-CoA transferase activity [GO:0033608] (molecular function) Definition: Catalysis of the reaction: formyl-CoA + oxalate = formate + oxalyl-CoA. Also known as: formyl-CoA oxalate CoA-transferase activity, formyl-CoA:oxalate CoA-transferase activity, formyl-coenzyme A transferase activity Relationships: is a type of GO:0008410 Sources: EC:2.8.3.16, RHEA:16545